{
  "gene_name": "Armadillo repeat-containing protein 2",
  "term_id": "UNKNOWN:0001",
  "gene": "UniProtKB:Q8NEN0",
  "term_label": "Unknown molecular function",
  "gene_symbol": "ARMC2"
}